{
  "term_label": "cysteine-type endopeptidase inhibitor activity",
  "gene": "UniProtKB:P09228",
  "gene_symbol": "CST2",
  "term_id": "GO:0004869",
  "gene_name": "Cystatin-SA"
}